{
  "term_label": "Unknown molecular function",
  "gene_name": "F-box and leucine-rich protein 22",
  "gene": "UniProtKB:Q6P050",
  "gene_symbol": "FBXL22",
  "term_id": "UNKNOWN:0001"
}